fibroblast growth factor receptor signaling pathway involved in forebrain neuron fate commitment [GO:0021899] (biological process) Definition: The series of molecular signals generated as a consequence of a fibroblast growth factor receptor binding to one of its physiological ligands that contributes to the commitment of a neuroblast to a neuronal fate. The neuron will reside in the forebrain. References: PMID:16226447 Sources: GOC:cls, GOC:dgh, GOC:dph, GOC:jid, GO_REF:0000021 Also known as: fibroblast growth factor receptor signalling pathway involved in forebrain neuron fate commitment Relationships: is a type of fibroblast growth factor receptor signaling pathway [GO:0008543]; is part of commitment of multipotent stem cells to neuronal lineage in forebrain [GO:0021898]